{
  "gene": "UniProtKB:Q9GZS3",
  "gene_symbol": "SKIC8",
  "gene_name": "Superkiller complex protein 8",
  "term_id": "UNKNOWN:0001",
  "term_label": "Unknown molecular function"
}